{
  "term_id": "GO:0000977",
  "gene_symbol": "RHOXF2B",
  "gene_name": "Rhox homeobox family member 2B",
  "term_label": "RNA polymerase II transcription regulatory region sequence-specific DNA binding",
  "gene": "UniProtKB:P0C7M4"
}